{
  "term_id": "GO:0005801",
  "term_label": "cis-Golgi network",
  "gene_name": "Golgin subfamily A member 8O",
  "gene_symbol": "GOLGA8O",
  "gene": "UniProtKB:A6NCC3"
}